dimethylamine methyltransferase activity [GO:0043791] (MF) Definition: Catalysis of the reaction: dimethylamine + a dimethylamine corrinoid protein = a methylated dimethylamine corrinoid protein + methylamine. Relationships: is a type of methyltransferase activity [GO:0008168] References: PMID:9874228 Note: This function is the first step in the pathway of methanogenesis from dimethylamine. Also known as: MT1, DMA methyltransferase 1, DMAMT 1, dimethylamine:corrinoid methyltransferase activity, dimethylamine-specific methylcobalamin:coenzyme M methyltransferase activity, mtbB1